{
  "term_id": "UNKNOWN:0001",
  "gene": "UniProtKB:A8MW99",
  "gene_name": "Meiosis-specific protein MEI4",
  "gene_symbol": "MEI4",
  "term_label": "Unknown molecular function"
}